{
  "gene": "UniProtKB:Q9ULX5",
  "term_label": "GTPase activity",
  "gene_symbol": "RNF112",
  "gene_name": "RING finger protein 112",
  "term_id": "GO:0003924"
}